dense nuclear body [GO:0046818] (cellular component) Relationships: is a type of cellular anatomical structure [GO:0110165]; is part of nucleus [GO:0005634] Definition: A location in the host cell nucleus where viral proteins colocalize late in infection prior to the onset of viral DNA synthesis. More than one site can be present simultaneously. References: PMID:10233976